{
  "gene": "UniProtKB:Q8NC56",
  "term_id": "GO:0005637",
  "gene_symbol": "LEMD2",
  "term_label": "nuclear inner membrane",
  "gene_name": "LEM domain-containing protein 2"
}